maintenance of unfolded protein [GO:0036506] (BP) References: PMID:21636303 Sources: GOC:BHF, GOC:PARL, GOC:bf, GOC:nc Subtypes: maintenance of unfolded protein involved in ERAD pathway [GO:1904378] Relationships: is a type of GO:0031647 Definition: Maintaining a protein in an unfolded, soluble state.